{
  "gene_name": "Apolipoprotein(a)",
  "term_label": "Unknown cellular component",
  "gene": "UniProtKB:P08519",
  "term_id": "UNKNOWN:0003",
  "gene_symbol": "LPA"
}